Sertoli cell development [GO:0060009] (biological process) Definition: The process whose specific outcome is the progression of a Sertoli cell over time, from its formation to the mature structure. Cell development does not include the steps involved in committing a cell to a Sertoli cell fate. Sources: GOC:dph Relationships: is a type of epithelial cell development [GO:0002064]; is a type of GO:0003006; is part of Sertoli cell differentiation [GO:0060008] Subtypes: establishment of Sertoli cell barrier [GO:0097368]